{
  "term_label": "antigen binding",
  "gene_symbol": "IGHV3OR16-10",
  "gene": "UniProtKB:A0A075B7F0",
  "gene_name": "Immunoglobulin heavy variable 3_OR16-10 (non-functional) (Fragment)",
  "term_id": "GO:0003823"
}